{
  "term_id": "GO:0043005",
  "gene_symbol": "CPEB3",
  "term_label": "neuron projection",
  "gene_name": "Cytoplasmic polyadenylation element-binding protein 3",
  "gene": "UniProtKB:Q8NE35"
}